{
  "term_label": "ASAP complex",
  "gene_name": "RNA-binding protein with serine-rich domain 1",
  "term_id": "GO:0061574",
  "gene_symbol": "RNPS1",
  "gene": "UniProtKB:Q15287"
}